{
  "gene_symbol": "CEBPZ",
  "gene": "UniProtKB:Q03701",
  "term_id": "UNKNOWN:0001",
  "term_label": "Unknown molecular function",
  "gene_name": "CCAAT_enhancer-binding protein zeta"
}